{
  "term_id": "GO:0005886",
  "term_label": "plasma membrane",
  "gene_symbol": "MET",
  "gene": "UniProtKB:P08581",
  "gene_name": "Hepatocyte growth factor receptor"
}